{
  "gene": "UniProtKB:Q9Y4X5",
  "term_label": "nucleus",
  "term_id": "GO:0005634",
  "gene_name": "E3 ubiquitin-protein ligase ARIH1",
  "gene_symbol": "ARIH1"
}